{
  "gene_name": "Late cornified envelope protein 3C",
  "term_label": "Unknown cellular component",
  "gene": "UniProtKB:Q5T5A8",
  "gene_symbol": "LCE3C",
  "term_id": "UNKNOWN:0003"
}